hyaluronate lyase activity [GO:0030340] (molecular function) Definition: Catalysis of the reaction: hyaluronate = n 3-(4-deoxy-beta-D-gluc-4-enuronosyl)-N-acetyl-D-glucosamine. Sources: EC:4.2.2.1 Also known as: hyaluronidase activity, glucuronoglycosaminoglycan lyase activity, hyaluronidase [but cf. EC:3.2.1.35 (hyalurononglucosaminidase) and EC:3.2.1.36 (hyaluronoglucuronidase)], mucinase activity, spreading factor activity Relationships: is a type of GO:0016837